{
  "term_label": "serine-type endopeptidase activity",
  "gene_symbol": "PCSK9",
  "gene_name": "Proprotein convertase subtilisin_kexin type 9",
  "term_id": "GO:0004252",
  "gene": "UniProtKB:Q8NBP7"
}